{
  "gene_name": "Synaptotagmin-8",
  "gene": "UniProtKB:Q8NBV8",
  "term_id": "GO:0031045",
  "gene_symbol": "SYT8",
  "term_label": "dense core granule"
}